{
  "gene_symbol": "ZNG1B",
  "gene": "UniProtKB:Q8IUF1",
  "term_id": "GO:0005737",
  "term_label": "cytoplasm",
  "gene_name": "Zinc-regulated GTPase metalloprotein activator 1B"
}